positive regulation of epithelial cell migration [GO:0010634] (biological process) Relationships: is a type of regulation of epithelial cell migration [GO:0010632]; is a type of positive regulation of cell migration [GO:0030335]; positively regulates epithelial cell migration [GO:0010631] Definition: Any process that activates or increases the frequency, rate or extent of epithelial cell migration. Sources: GOC:BHF, GOC:dph, GOC:tb Subtypes: positive regulation of keratinocyte migration [GO:0051549], GO:1903688